{
  "gene_symbol": "SEMG1",
  "gene_name": "Semenogelin-1",
  "term_id": "GO:0005615",
  "term_label": "extracellular space",
  "gene": "UniProtKB:P04279"
}